dynorphin receptor activity [GO:0038048] (molecular function) Sources: GOC:bf, Wikipedia:Dynorphin Also known as: kappa-opioid receptor activity Relationships: is a type of GO:0004985; is a type of G protein-coupled peptide receptor activity [GO:0008528] Definition: Combining with a dynorphin peptide, and transmitting the signal across the membrane by activating an associated G-protein. Dynorphin is any opioid peptide that is generated by cleavage of the precursor protein prodynorphin.